{
  "gene_name": "Disks large homolog 1",
  "gene_symbol": "DLG1",
  "term_id": "GO:0007399",
  "gene": "UniProtKB:Q12959",
  "term_label": "nervous system development"
}